{
  "term_label": "protein import into mitochondrial matrix",
  "gene_symbol": "DNLZ",
  "gene": "UniProtKB:Q5SXM8",
  "gene_name": "DNL-type zinc finger protein",
  "term_id": "GO:0030150"
}